activation-induced cell death of T cells [GO:0006924] (biological process) Definition: A T cell apoptotic process that occurs towards the end of the expansion phase following the initial activation of mature T cells by antigen and is triggered by T cell receptor stimulation and signals transmitted via various surface-expressed members of the TNF receptor family such as Fas ligand, Fas, and TNF and the p55 and p75 TNF receptors. Also known as: AICD, activated T cell apoptosis, antigen-driven apoptosis, activation-induced cell death of T lymphocytes, activation-induced cell death of T-cells, activation-induced cell death of T-lymphocytes References: PMID:12414721, PMID:12752672 Sources: GOC:add, GOC:mtg_apoptosis, ISBN:0781765196 Relationships: is_a T cell apoptotic process [GO:0070231]; BFO_0000050 GO:0043029 Regulation: regulated by regulation of activation-induced cell death of T cells [GO:0070235]; negatively regulated by negative regulation of activation-induced cell death of T cells [GO:0070236]; positively regulated by GO:0070237